{
  "gene_name": "POU domain, class 3, transcription factor 4",
  "term_label": "regulation of transcription by RNA polymerase II",
  "gene_symbol": "POU3F4",
  "gene": "UniProtKB:P49335",
  "term_id": "GO:0006357"
}